{
  "gene": "UniProtKB:P08123",
  "gene_symbol": "COL1A2",
  "gene_name": "Collagen alpha-2(I) chain",
  "term_id": "GO:0043588",
  "term_label": "skin development"
}